eukaryotic translation elongation factor 1 complex [GO:0005853] (cellular component) References: PMID:10216950 Sources: GOC:jl Definition: A multisubunit nucleotide exchange complex that binds GTP and aminoacyl-tRNAs, and catalyzes their codon-dependent placement at the A-site of the ribosome. In humans, the complex is composed of four subunits, alpha, beta, delta and gamma. Relationships: is a type of protein-containing complex [GO:0032991]; is part of GO:0005737